{
  "term_label": "mitochondrion organization",
  "gene_symbol": "ADCK1",
  "gene_name": "AarF domain-containing protein kinase 1",
  "gene": "UniProtKB:Q86TW2",
  "term_id": "GO:0007005"
}